{
  "gene_symbol": "C9orf50",
  "term_id": "UNKNOWN:0001",
  "gene_name": "Uncharacterized protein C9orf50",
  "gene": "UniProtKB:Q5SZB4",
  "term_label": "Unknown molecular function"
}